NAD+-histone H2BS6 serine ADP-ribosyltransferase activity [GO:0140816] (molecular function) Note: Note that the residue position corresponds to the canonical human H2B histone (UniProtKB:P62807); the N-terminus of histone H2B is divergent across eukaryotes; make sure that the paper clearly references the human protein for the position of this modification to use this term. Residue 1 is the first residue following removal of the initiating Methionine (Met). Note that each histone is encoded by multiple genes, and sequences may vary across different genes within an organism. Also known as: NAD+-histone H2B-S6 serine ADP-ribosyltransferase activity, NAD+-histone-serine ADP-ribosyltransferase activity (H2B-S6 specific) Relationships: is a type of NAD+-protein-serine ADP-ribosyltransferase activity [GO:0140805] Definition: Catalysis of the transfer of ADP-ribose groups to the serine-6 or an equivalent residue of the N-terminal tail of histone H2B. References: PMID:34874266